{
  "gene_name": "Potassium channel subfamily K member 12",
  "term_id": "GO:0071805",
  "gene_symbol": "KCNK12",
  "gene": "UniProtKB:Q9HB15",
  "term_label": "potassium ion transmembrane transport"
}